{
  "gene": "UniProtKB:Q8N2M8",
  "term_label": "Unknown molecular function",
  "term_id": "UNKNOWN:0001",
  "gene_symbol": "CLASRP",
  "gene_name": "CLK4-associating serine_arginine rich protein"
}